{
  "gene_symbol": "ERBB4",
  "gene_name": "Receptor tyrosine-protein kinase erbB-4",
  "gene": "UniProtKB:Q15303",
  "term_id": "GO:0009925",
  "term_label": "basal plasma membrane"
}